mitochondrial 5'-adenylyl sulfate transmembrane transport [GO:1990553] (biological process) References: PMID:24296033 Definition: The process in which 5'-adenylyl sulfate is transported across a mitochondrial membrane, into or out of the mitochondrion. Relationships: is a type of GO:1902558